protein methyltransferase activity [GO:0008276] (molecular function) Subtypes: methylated-DNA-[protein]-cysteine S-methyltransferase activity [GO:0003908], diphthine synthase activity [GO:0004164], protein-arginine N-methyltransferase activity [GO:0016274], GO:0016279, protein-L-histidine N-tele-methyltransferase activity [GO:0018064], protein-arginine C-methyltransferase activity [GO:0035244], protein-glutamine N-methyltransferase activity [GO:0036009], histone methyltransferase activity [GO:0042054], protein carboxyl O-methyltransferase activity [GO:0051998], N-terminal protein N-methyltransferase activity [GO:0071885], protein-cysteine methyltransferase activity [GO:0106363], protein-L-histidine N-pros-methyltransferase activity [GO:0106370], diphthine methyl ester synthase activity [GO:0141133] Also known as: protein methylase activity Sources: GOC:jl Relationships: is a type of methyltransferase activity [GO:0008168]; is a type of catalytic activity, acting on a protein [GO:0140096] Definition: Catalysis of the transfer of a methyl group (CH3-) to a protein.